{
  "gene_symbol": "MRAS",
  "term_id": "GO:0003924",
  "gene_name": "Ras-related protein M-Ras",
  "gene": "UniProtKB:O14807",
  "term_label": "GTPase activity"
}